{
  "gene": "UniProtKB:Q16236",
  "term_label": "DNA-binding transcription factor activity, RNA polymerase II-specific",
  "gene_name": "Nuclear factor erythroid 2-related factor 2",
  "gene_symbol": "NFE2L2",
  "term_id": "GO:0000981"
}